{
  "term_id": "GO:0071568",
  "term_label": "UFM1 transferase activity",
  "gene_name": "E3 UFM1-protein ligase 1",
  "gene": "UniProtKB:O94874",
  "gene_symbol": "UFL1"
}